{
  "term_id": "GO:0000723",
  "gene": "UniProtKB:O94761",
  "gene_symbol": "RECQL4",
  "gene_name": "ATP-dependent DNA helicase Q4",
  "term_label": "telomere maintenance"
}